{
  "term_label": "tRNA binding",
  "term_id": "GO:0000049",
  "gene": "UniProtKB:O60524",
  "gene_symbol": "NEMF",
  "gene_name": "Ribosome quality control complex subunit NEMF"
}